{
  "term_label": "gamma-aminobutyric acid:sodium:chloride symporter activity",
  "term_id": "GO:0005332",
  "gene_name": "Sodium- and chloride-dependent betaine transporter",
  "gene_symbol": "SLC6A12",
  "gene": "UniProtKB:P48065"
}